{
  "gene": "UniProtKB:Q6UXV4",
  "term_label": "MICOS complex",
  "gene_symbol": "APOOL",
  "gene_name": "MICOS complex subunit MIC27",
  "term_id": "GO:0061617"
}